pronephros development [GO:0048793] (biological process) Definition: The process whose specific outcome is the progression of the pronephros over time, from its formation to the mature structure. In mammals, the pronephros is the first of the three embryonic kidneys to be established and exists only transiently. In lower vertebrates such as fish and amphibia, the pronephros is the fully functional embryonic kidney and is indispensable for larval life. References: PMID:10535314, PMID:15968585, PMID:18322540 Sources: GOC:bf, GOC:mtg_kidney_jan10, XAO:00002000, ZFA:0000151 Also known as: pronephric kidney development Relationships: is a type of GO:0001822 Subtypes: head kidney development [GO:0072113]